petal vascular tissue pattern formation [GO:0080056] (biological process) Definition: Vascular tissue pattern formation as it occurs in the petal of vascular plants. References: PMID:17369435 Relationships: is a type of GO:0010051